{
  "gene_symbol": "ACY3",
  "term_label": "aminoacylase activity",
  "gene_name": "N-acyl-aromatic-L-amino acid amidohydrolase (carboxylate-forming)",
  "term_id": "GO:0004046",
  "gene": "UniProtKB:Q96HD9"
}